{
  "term_id": "GO:1990756",
  "gene": "UniProtKB:Q9NR64",
  "gene_symbol": "KLHL1",
  "gene_name": "Kelch-like protein 1",
  "term_label": "ubiquitin-like ligase-substrate adaptor activity"
}